CMP-N-acylneuraminate phosphodiesterase activity [GO:0047392] (molecular function) Also known as: CMP-N-acetylneuraminate hydrolase activity, CMP-N-acylneuraminate N-acylneuraminohydrolase activity, CMP-N-acylneuraminic acid hydrolase activity, CMP-sialate hydrolase activity, CMP-sialic acid hydrolase activity, cytidine monophosphate-N-acetylneuraminic acid hydrolase activity, cytidine monophosphosialate hydrolase activity, cytidine monophosphosialic hydrolase activity Relationships: is a type of GO:0008081 Definition: Catalysis of the reaction: H2O + CMP-N-acylneuraminate = N-acylneuraminate + CMP. Sources: EC:3.1.4.40, MetaCyc:3.1.4.40-RXN